{
  "gene": "UniProtKB:Q96L50",
  "gene_name": "Leucine-rich repeat protein 1",
  "gene_symbol": "LRR1",
  "term_label": "Unknown cellular component",
  "term_id": "UNKNOWN:0003"
}